sister chromatid cohesion [GO:0007062] (biological process) Definition: The cell cycle process in which the sister chromatids of a replicated chromosome become tethered to each other. Relationships: is a type of GO:0022402; is a type of chromosome organization [GO:0051276] Subtypes: mitotic sister chromatid cohesion [GO:0007064], meiotic sister chromatid cohesion [GO:0051177], centromeric sister chromatid cohesion [GO:0070601] Also known as: cohesion-mediated DNA tethering Sources: GOC:jh, GOC:mah, ISBN:0815316194 Regulation: regulated by regulation of sister chromatid cohesion [GO:0007063]; negatively regulated by negative regulation of sister chromatid cohesion [GO:0045875]; positively regulated by positive regulation of sister chromatid cohesion [GO:0045876]